appendage development [GO:0048736] (biological process) Relationships: is a type of GO:0048856; is part of multicellular organism development [GO:0007275] Sources: GOC:jid, GOC:rc Subtypes: fin development [GO:0033333], imaginal disc-derived appendage development [GO:0048737], limb development [GO:0060173] Definition: The process whose specific outcome is the progression of an appendage over time, from its formation to the mature structure. An appendage is an organ or part that is attached to the trunk of an organism, such as a limb or a branch.